detection of fungus [GO:0016046] (biological process) Relationships: is a type of GO:0009620; is a type of detection of other organism [GO:0098543] Also known as: detection of fungi, detection of parasitic fungi, detection of parasitic fungus, perception of parasitic fungi, perception of fungi, perception of fungus, perception of parasitic fungus Sources: GOC:hb Definition: The series of events in which a stimulus from a fungus is received and converted into a molecular signal. Subtypes: detection of yeast [GO:0001879], GO:0009603